{
  "term_id": "UNKNOWN:0001",
  "gene_name": "Roundabout homolog 2",
  "term_label": "Unknown molecular function",
  "gene": "UniProtKB:Q9HCK4",
  "gene_symbol": "ROBO2"
}